{
  "term_id": "GO:0005737",
  "gene_name": "Cyclin-A1",
  "term_label": "cytoplasm",
  "gene": "UniProtKB:P78396",
  "gene_symbol": "CCNA1"
}